senecionine N-oxygenase activity [GO:0033784] (molecular function) Relationships: is a type of oxidoreductase activity, acting on paired donors, with incorporation or reduction of molecular oxygen, NAD(P)H as one donor, and incorporation of one atom of oxygen [GO:0016709] Sources: EC:1.14.13.101, RHEA:11420 Also known as: SNO, senecionine monooxygenase (N-oxide-forming) activity, senecionine,NADPH:oxygen oxidoreductase (N-oxide-forming) activity Definition: Catalysis of the reaction: H+ + NADPH + O2 + senecionine = H2O + NADP+ + senecionine N-oxide.